vitamin D3 catabolic process [GO:1901754] (biological process) Definition: The chemical reactions and pathways resulting in the breakdown of vitamin D3. Sources: GOC:TermGenie, GOC:yaf Also known as: calciol breakdown, calciol catabolic process, calciol catabolism, calciol degradation, cholecalciferol catabolic process, cholecalciferol catabolism, vitamin D3 breakdown, vitamin D3 catabolism, vitamin D3 degradation Relationships: is a type of vitamin D catabolic process [GO:0042369]; is a type of alcohol catabolic process [GO:0046164]; is a type of vitamin D3 metabolic process [GO:0070640]